steviolbioside glucosyltransferase activity (stevioside forming) [GO:0102379] (molecular function) Sources: RHEA:61744 Relationships: is a type of hexosyltransferase activity [GO:0016758] Definition: Catalysis of the reaction: steviolbioside + UDP-alpha-D-glucose = stevioside + UDP.